{
  "term_label": "blood coagulation, intrinsic pathway",
  "gene_name": "Platelet glycoprotein V",
  "term_id": "GO:0007597",
  "gene": "UniProtKB:P40197",
  "gene_symbol": "GP5"
}